dense core granule cytoskeletal transport [GO:0099519] (biological process) Definition: The directed movement of dense core granules along cytoskeletal fibers, such as microtubules or actin filaments. References: PMID:23358451 Sources: GOC:kmv Also known as: dense core vesicle cytoskeletal trafficking Relationships: is a type of vesicle cytoskeletal trafficking [GO:0099518]; is a type of dense core granule transport [GO:1901950]; occurs in GO:0030424 Subtypes: anterograde neuronal dense core vesicle transport [GO:1990048], retrograde neuronal dense core vesicle transport [GO:1990049]